{
  "gene": "UniProtKB:Q9BQS2",
  "term_id": "GO:0017158",
  "gene_name": "Synaptotagmin-15",
  "gene_symbol": "SYT15",
  "term_label": "regulation of calcium ion-dependent exocytosis"
}